{
  "term_label": "steroid metabolic process",
  "gene_name": "Retinol dehydrogenase 5",
  "term_id": "GO:0008202",
  "gene": "UniProtKB:Q92781",
  "gene_symbol": "RDH5"
}